{
  "term_id": "UNKNOWN:0002",
  "gene_symbol": "C5orf47",
  "term_label": "Unknown biological process",
  "gene": "UniProtKB:Q569G3",
  "gene_name": "Uncharacterized protein C5orf47"
}